3-hydroxybenzoate 2-monooxygenase activity [GO:0047563] (molecular function) Definition: Catalysis of the reaction: 3-hydroxybenzoate + AH(2) + O2 = 2,3-dihydroxybenzoate + A + H2O. Also known as: 3-hydroxybenzoate 2-hydroxylase activity, 3-HBA-2-hydroxylase activity, 3-hydroxybenzoate,hydrogen-donor:oxygen oxidoreductase (2-hydroxylating) Relationships: is a type of GO:0004497; is a type of oxidoreductase activity, acting on paired donors, with incorporation or reduction of molecular oxygen [GO:0016705] Sources: EC:1.14.99.23, RHEA:14193